{
  "gene_symbol": "DENND4B",
  "term_id": "GO:0032483",
  "gene": "UniProtKB:O75064",
  "term_label": "regulation of Rab protein signal transduction",
  "gene_name": "DENN domain-containing protein 4B"
}